{
  "term_label": "fructose metabolic process",
  "term_id": "GO:0006000",
  "gene": "UniProtKB:P50053",
  "gene_symbol": "KHK",
  "gene_name": "Ketohexokinase"
}